{
  "gene_symbol": "NOS2",
  "term_id": "GO:0006954",
  "gene_name": "Nitric oxide synthase, inducible",
  "term_label": "inflammatory response",
  "gene": "UniProtKB:P35228"
}